{
  "gene_symbol": "RGS1",
  "gene": "UniProtKB:Q08116",
  "gene_name": "Regulator of G-protein signaling 1",
  "term_id": "GO:0045744",
  "term_label": "negative regulation of G protein-coupled receptor signaling pathway"
}